positive regulation of isotype switching to IgD isotypes [GO:0048301] (biological process) Definition: Any process that activates or increases the frequency, rate or extent of isotype switching to IgD isotypes. Sources: GOC:jid Relationships: is a type of positive regulation of isotype switching [GO:0045830]; is a type of regulation of isotype switching to IgD isotypes [GO:0048299]; positively regulates isotype switching to IgD isotypes [GO:0048292] Also known as: positive regulation of class switch recombination to IgD isotypes, positive regulation of class switching to IgD isotypes, positive regulation of isotype switch recombination to IgD isotypes, up regulation of isotype switching to IgD isotypes, up-regulation of isotype switching to IgD isotypes, upregulation of isotype switching to IgD isotypes, activation of isotype switching to IgD isotypes, stimulation of isotype switching to IgD isotypes